negative regulation of mitotic division septum assembly [GO:0140280] (biological process) Relationships: is a type of negative regulation of division septum assembly [GO:0010974]; is a type of regulation of mitotic division septum assembly [GO:0140279]; is a type of negative regulation of mitotic cytokinetic process [GO:1903437]; negatively regulates mitotic division septum assembly [GO:0140278] References: PMID:22786806 Subtypes: negative regulation of secondary cell septum biogenesis [GO:1903396], negative regulation of primary cell septum biogenesis [GO:1905757] Also known as: down regulation of division septum formation involved in mitotic cell cycle, down regulation of formation of division septum involved in mitotic cell cycle, down regulation of mitotic division septum assembly, down regulation of septin assembly and septum biosynthesis involved in mitotic cell cycle, down regulation of septin assembly and septum formation involved in mitotic cell cycle, down-regulation of division septum formation involved in mitotic cell cycle, down-regulation of formation of division septum involved in mitotic cell cycle, down-regulation of mitotic division septum assembly, down-regulation of septin assembly and septum biosynthesis involved in mitotic cell cycle, down-regulation of septin assembly and septum formation involved in mitotic cell cycle, downregulation of division septum formation involved in mitotic cell cycle, downregulation of formation of division septum involved in mitotic cell cycle, downregulation of mitotic division septum assembly, downregulation of septin assembly and septum biosynthesis involved in mitotic cell cycle, downregulation of septin assembly and septum formation involved in mitotic cell cycle, inhibition of septin assembly and septum biosynthesis involved in mitotic cell cycle, inhibition of septin assembly and septum formation involved in mitotic cell cycle, negative regulation of division septum formation involved in mitotic cell cycle, negative regulation of formation of division septum involved in mitotic cell cycle, negative regulation of septin assembly and septum biosynthesis involved in mitotic cell cycle, negative regulation of septin assembly and septum formation involved in mitotic cell cycle, inhibition of division septum formation involved in mitotic cell cycle, inhibition of formation of division septum involved in mitotic cell cycle, inhibition of mitotic division septum assembly Definition: Any process that stops, prevents or reduces the frequency, rate or extent of mitotic division septum formation. Division septum formation is the assembly and arrangement of a septum that spans the plasma membrane interface between progeny cells following cytokinesis.